{
  "gene_symbol": "ARHGEF19",
  "term_label": "wound healing",
  "gene": "UniProtKB:Q8IW93",
  "term_id": "GO:0042060",
  "gene_name": "Rho guanine nucleotide exchange factor 19"
}